allantoate transmembrane transporter activity [GO:0015124] (molecular function) Definition: Enables the transfer of allantoate from one side of a membrane to the other. Allantoate is the end product of purine metabolism in mammals and some fish, formed form allantoin. It is widely distributed in plants as an important source of stored nitrogen. Sources: GOC:ai, ISBN:0198547684 Relationships: is a type of amide transmembrane transporter activity [GO:0042887]; is a type of carboxylic acid transmembrane transporter activity [GO:0046943]; is part of GO:0015719